metanephric nephron epithelium development [GO:0072243] (biological process) Definition: The process whose specific outcome is the progression of the metanephric nephron epithelium over time, from its formation to the mature structure. An epithelium is a tissue that covers the internal or external surfaces of an anatomical structure. The metanephric nephron epithelium is a tissue that covers the surface of a nephron in the metanephros. Subtypes: metanephric early distal convoluted tubule development [GO:0072222], metanephric late distal convoluted tubule development [GO:0072225], metanephric macula densa development [GO:0072227], metanephric nephron tubule development [GO:0072234], GO:0072244, metanephric long descending thin limb development [GO:0072269], metanephric short descending thin limb development [GO:0072271] Sources: GOC:mtg_kidney_jan10 Relationships: is a type of GO:0072009; is a type of metanephric epithelium development [GO:0072207]